melanocyte-stimulating hormone activity [GO:0017044] (molecular function) Sources: ISBN:0198506732 Also known as: melanocyte stimulating hormone activity, alpha-melanocyte stimulating hormone activity, alpha-melanophore stimulating hormone activity Relationships: is a type of GO:0005179 Definition: The action characteristic of melanocyte-stimulating hormone, any of three peptide hormones that are produced by the intermediate lobe of the pituitary gland and, upon receptor binding, cause dispersal of melanosomes in melanophores of poikilothermic vertebrates.